{
  "term_label": "plasma membrane",
  "term_id": "GO:0005886",
  "gene_symbol": "ADAP1",
  "gene": "UniProtKB:O75689",
  "gene_name": "Arf-GAP with dual PH domain-containing protein 1"
}